{
  "gene_symbol": "FGF1",
  "term_id": "GO:0005737",
  "gene_name": "Fibroblast growth factor 1",
  "term_label": "cytoplasm",
  "gene": "UniProtKB:P05230"
}